{
  "term_label": "Unknown cellular component",
  "term_id": "UNKNOWN:0003",
  "gene_symbol": "ZMYM1",
  "gene_name": "Zinc finger MYM-type protein 1",
  "gene": "UniProtKB:Q5SVZ6"
}